virus tail, tip [GO:0098023] (cellular component) Definition: The basal end of the virus tail, which is used by the virus to attach to the host cell. Also known as: bacteriophage tail tip Relationships: is a type of virion component [GO:0044423]; is part of virus tail [GO:0098015] Sources: GOC:bm